glial cell-derived neurotrophic factor production [GO:0044467] (biological process) Definition: The regulated release of glial cell line-derived neurotrophic factor from a cell. Glial cell-derived neurotrophic factor (GDNF) is a small protein that potently promotes the survival of many types of neurons, notably dopaminergic and motor neurons. References: PMID:17505307 Sources: GOC:yaf Also known as: GDNF production, glial cell-derived neurotrophic factor secretion, glial cell line-derived neurotrophic factor production Relationships: is a type of cytokine production [GO:0001816] Regulation: regulated by GO:1900166; negatively regulated by negative regulation of glial cell-derived neurotrophic factor production [GO:1900167]; positively regulated by positive regulation of glial cell-derived neurotrophic factor production [GO:1900168]